{
  "term_id": "GO:0030198",
  "term_label": "extracellular matrix organization",
  "gene": "UniProtKB:Q9H306",
  "gene_name": "Matrix metalloproteinase-27",
  "gene_symbol": "MMP27"
}